magnesium ion transport [GO:0015693] (biological process) Relationships: is a type of GO:0030001 Also known as: magnesium transport Sources: GOC:ai Definition: The directed movement of magnesium (Mg) ions into, out of or within a cell, or between cells, by means of some agent such as a transporter or pore. Subtypes: magnesium ion transmembrane transport [GO:1903830]